aspartate-ammonia ligase (ADP-forming) activity [GO:0047478] (molecular function) Relationships: is a type of acid-ammonia (or amide) ligase activity [GO:0016880] Sources: EC:6.3.1.4, RHEA:14197 Also known as: L-aspartate:ammonia ligase (ADP-forming), asparagine synthetase (ADP-forming) activity, asparagine synthetase (adenosine diphosphate-forming) Definition: Catalysis of the reaction: L-aspartate + ATP + NH4 = L-asparagine + ADP + 2 H+ + phosphate.